{
  "gene_name": "Tripartite motif-containing protein 43",
  "term_id": "GO:0005737",
  "gene_symbol": "TRIM43",
  "gene": "UniProtKB:Q96BQ3",
  "term_label": "cytoplasm"
}